{
  "term_id": "GO:0000978",
  "gene_name": "Tumor protein 63",
  "gene": "UniProtKB:Q9H3D4",
  "gene_symbol": "TP63",
  "term_label": "RNA polymerase II cis-regulatory region sequence-specific DNA binding"
}